postsynaptic specialization [GO:0099572] (cellular component) Definition: A network of proteins within and adjacent to the postsynaptic membrane. Its major components include neurotransmitter receptors and the proteins that spatially and functionally organize them such as anchoring and scaffolding molecules, signaling enzymes and cytoskeletal components. References: PMID:22046028 Relationships: is a type of GO:0043226; is part of postsynapse [GO:0098794] Subtypes: postsynaptic density [GO:0014069], muscle cell postsynaptic specialization [GO:0097482], postsynaptic specialization of symmetric synapse [GO:0099629]